{
  "gene_symbol": "UNG",
  "term_label": "nucleus",
  "gene": "UniProtKB:P13051",
  "gene_name": "Uracil-DNA glycosylase",
  "term_id": "GO:0005634"
}